amniotic stem cell differentiation [GO:0097086] (biological process) Regulation: regulated by regulation of amniotic stem cell differentiation [GO:2000797]; negatively regulated by negative regulation of amniotic stem cell differentiation [GO:2000798]; positively regulated by positive regulation of amniotic stem cell differentiation [GO:2000799] Definition: The process whereby a relatively unspecialized cell acquires specialized features of an amniotic stem cell. An amniotic stem cell is a mesenchymal stem cell extracted from amniotic fluid. Amniotic stem cells are able to differentiate into various tissue types such as skin, cartilage, cardiac tissue, nerves, muscle, and bone. References: PMID:20942606 Sources: CL:0002639, GOC:yaf, Wikipedia:Amniotic_stem_cells Relationships: is a type of mesenchymal stem cell differentiation [GO:0072497]